{
  "gene_name": "Dual specificity testis-specific protein kinase 2",
  "gene": "UniProtKB:Q96S53",
  "gene_symbol": "TESK2",
  "term_label": "cytoplasm",
  "term_id": "GO:0005737"
}